{
  "gene": "UniProtKB:Q8NFJ8",
  "term_id": "GO:0007423",
  "gene_symbol": "BHLHE22",
  "gene_name": "Class E basic helix-loop-helix protein 22",
  "term_label": "sensory organ development"
}